{
  "term_label": "myofibril",
  "gene": "UniProtKB:P28289",
  "gene_symbol": "TMOD1",
  "gene_name": "Tropomodulin-1",
  "term_id": "GO:0030016"
}